{
  "gene": "UniProtKB:P60371",
  "term_label": "Unknown biological process",
  "gene_name": "Keratin-associated protein 10-6",
  "gene_symbol": "KRTAP10-6",
  "term_id": "UNKNOWN:0002"
}